HSP90-CDC37 chaperone complex [GO:1990565] (CC) Relationships: is a type of protein folding chaperone complex [GO:0101031]; is part of cytoplasm [GO:0005737] Definition: A protein kinase chaperone complex required for the proper folding, maturation and stabilization of target proteins (mostly signaling protein kinases, some steroid hormone receptors), usually during or immediately after completion of translation. The highly conserved, phosphorylated CDC37-Ser13 (vertebrates) or cdc37-Ser14 (yeast) is essential for complex assembly and target protein binding. CDC37-Ser13 (Ser14) is phosphorylated by Casein kinase II (CK2), which in turn is a target of CDC37 creating a positive feedback loop. Complex binding also prevents rapid ubiquitin-dependent proteosomal degradation of target proteins. References: PMID:21855797, PMID:22939624 Sources: GOC:PARL, GOC:bhm, GOC:pad Note: An example of this is HSP90AB1 in human (UniProt symbol P08238) in PMID:21855797 (inferred from direct assay).